{
  "gene_name": "Prefoldin subunit 4",
  "gene_symbol": "PFDN4",
  "term_label": "cytoplasm",
  "gene": "UniProtKB:Q9NQP4",
  "term_id": "GO:0005737"
}